{
  "gene": "UniProtKB:O95256",
  "gene_name": "Interleukin-18 receptor accessory protein",
  "gene_symbol": "IL18RAP",
  "term_label": "cell surface",
  "term_id": "GO:0009986"
}